brexanolone catabolic process [GO:0062175] (biological process) Definition: The chemical reactions and pathways resulting in the breakdown of brexanolone. Relationships: is a type of steroid catabolic process [GO:0006706]; is a type of ketone catabolic process [GO:0042182]; is a type of GO:0062173 References: PMID:24390875 Also known as: allopregnanolone breakdown, allopregnanolone catabolic process, allopregnanolone catabolism, allopregnanolone degradation, allotetrahydroprogesterone breakdown, allotetrahydroprogesterone catabolic process, allotetrahydroprogesterone catabolism, allotetrahydroprogesterone degradation, brexanolone breakdown, brexanolone catabolism, brexanolone degradation